{
  "gene": "UniProtKB:P35408",
  "term_label": "cellular response to prostaglandin E stimulus",
  "gene_name": "Prostaglandin E2 receptor EP4 subtype",
  "term_id": "GO:0071380",
  "gene_symbol": "PTGER4"
}